aminobutyraldehyde dehydrogenase (NAD+) activity [GO:0019145] (molecular function) Definition: Catalysis of the reaction: 4-aminobutanal + NAD+ + H2O = 4-aminobutanoate + NADH + 2 H+. Sources: EC:1.2.1.19 Also known as: 4-aminobutanal dehydrogenase activity, 4-aminobutanal:NAD+ 1-oxidoreductase activity, 4-aminobutyraldehyde dehydrogenase activity, ABAL dehydrogenase activity, gamma-aminobutyraldehyde dehydroganase activity Relationships: is a type of aldehyde dehydrogenase (NAD+) activity [GO:0004029]